positive regulation of fibroblast migration [GO:0010763] (biological process) Relationships: is a type of regulation of fibroblast migration [GO:0010762]; is a type of positive regulation of cell migration [GO:0030335]; positively regulates fibroblast migration [GO:0010761] Sources: GOC:BHF, GOC:dph, GOC:tb Definition: Any process that increases the rate, frequency or extent of fibroblast cell migration. Fibroblast cell migration is accomplished by extension and retraction of a pseudopodium. Also known as: positive regulation of fibroblast cell migration Subtypes: positive regulation of hepatic stellate cell migration [GO:0061870]